{
  "term_label": "G protein-coupled receptor signaling pathway",
  "gene": "UniProtKB:O95800",
  "gene_name": "Probable G-protein coupled receptor 75",
  "term_id": "GO:0007186",
  "gene_symbol": "GPR75"
}